mitotic actomyosin contractile ring [GO:0110085] (cellular component) References: PMID:27505246 Sources: GOC:vw Definition: A cytoskeletal structure composed of actin filaments, myosin, and myosin-associated proteins that forms beneath the plasma membrane of many cells, including animal cells and yeast cells, in a plane perpendicular to the axis of the mitotic spindle, i.e. the cell division plane. Ring contraction is associated with centripetal growth of the membrane that divides the cytoplasm of the two future daughter cells. In animal cells, the mitotic contractile ring is located inside the plasma membrane at the location of the cleavage furrow. In budding fungal cells, e.g. mitotic S. cerevisiae cells, the mitotic contractile ring forms beneath the plasma membrane at the mother-bud neck before mitosis. Relationships: is a type of actomyosin contractile ring [GO:0005826] Subtypes: cellular bud neck contractile ring [GO:0000142]